{
  "gene_name": "GRB2-related adapter protein-like",
  "gene": "UniProtKB:Q8TC17",
  "term_id": "GO:0035591",
  "term_label": "signaling adaptor activity",
  "gene_symbol": "GRAPL"
}